{
  "term_label": "Unknown molecular function",
  "gene_symbol": "INSIG2",
  "gene_name": "Insulin-induced gene 2 protein",
  "gene": "UniProtKB:Q9Y5U4",
  "term_id": "UNKNOWN:0001"
}